{
  "term_label": "mitochondrion organization",
  "gene_name": "LETM1 domain-containing protein LETM2, mitochondrial",
  "term_id": "GO:0007005",
  "gene": "UniProtKB:Q2VYF4",
  "gene_symbol": "LETM2"
}